{
  "gene": "UniProtKB:P34931",
  "term_label": "protein refolding",
  "gene_name": "Heat shock 70 kDa protein 1-like",
  "gene_symbol": "HSPA1L",
  "term_id": "GO:0042026"
}